{
  "gene_symbol": "FCRLA",
  "term_label": "transmembrane signaling receptor activity",
  "gene_name": "Fc receptor-like A",
  "term_id": "GO:0004888",
  "gene": "UniProtKB:Q7L513"
}